detection of chemical stimulus involved in sensory perception of taste [GO:0050912] (biological process) Definition: The series of events involved in the perception of taste in which a gustatory chemical stimulus is received and converted into a molecular signal. Sources: GOC:ai Also known as: taste perception, perception of taste, detection of chemical stimulus, perception of taste, sensory detection of chemical stimulus, perception of taste, sensory transduction of chemical stimulus, sensory detection of chemical stimulus during perception of taste, sensory detection of taste, sensory transduction of chemical stimulus during perception of taste, sensory transduction of taste Relationships: is a type of detection of chemical stimulus involved in sensory perception [GO:0050907]; is part of sensory perception of taste [GO:0050909] Subtypes: GO:0001580, detection of chemical stimulus involved in sensory perception of sour taste [GO:0001581], detection of chemical stimulus involved in sensory perception of sweet taste [GO:0001582], detection of chemical stimulus involved in sensory perception of salty taste [GO:0001583], detection of chemical stimulus involved in sensory perception of umami taste [GO:0046535]